{
  "term_label": "structural constituent of ribosome",
  "gene_symbol": "MRPL23",
  "term_id": "GO:0003735",
  "gene_name": "Large ribosomal subunit protein uL23m",
  "gene": "UniProtKB:Q16540"
}